{
  "gene_name": "ATP-dependent RNA helicase DDX19B",
  "gene_symbol": "DDX19B",
  "gene": "UniProtKB:Q9UMR2",
  "term_label": "RNA helicase activity",
  "term_id": "GO:0003724"
}